{
  "gene": "UniProtKB:O43683",
  "gene_symbol": "BUB1",
  "gene_name": "Mitotic checkpoint serine_threonine-protein kinase BUB1",
  "term_id": "GO:0051754",
  "term_label": "meiotic sister chromatid cohesion, centromeric"
}